{
  "gene_symbol": "HIGD2A",
  "term_label": "mitochondrion",
  "term_id": "GO:0005739",
  "gene": "UniProtKB:Q9BW72",
  "gene_name": "HIG1 domain family member 2A, mitochondrial"
}